{
  "term_id": "GO:0005886",
  "term_label": "plasma membrane",
  "gene": "UniProtKB:P08172",
  "gene_symbol": "CHRM2",
  "gene_name": "Muscarinic acetylcholine receptor M2"
}